{
  "term_label": "cell-cell adhesion mediator activity",
  "gene": "UniProtKB:Q8WZ75",
  "gene_symbol": "ROBO4",
  "term_id": "GO:0098632",
  "gene_name": "Roundabout homolog 4"
}